{
  "gene_name": "Zinc finger protein 169",
  "term_id": "GO:0005634",
  "gene_symbol": "ZNF169",
  "term_label": "nucleus",
  "gene": "UniProtKB:Q14929"
}